adenine deaminase activity [GO:0000034] (molecular function) Sources: RHEA:23688 Definition: Catalysis of the reaction: adenine + H+ + H2O = hypoxanthine + NH4+. Relationships: is a type of GO:0016814; is a type of deaminase activity [GO:0019239] Also known as: ADase activity, adenase activity, adenine aminase activity, adenine aminohydrolase activity